{
  "gene_name": "Amphoterin-induced protein 1",
  "term_label": "positive regulation of synapse assembly",
  "gene": "UniProtKB:Q86WK6",
  "gene_symbol": "AMIGO1",
  "term_id": "GO:0051965"
}